positive regulation of muscle tissue development [GO:1901863] (biological process) References: PMID:23150719 Sources: GOC:TermGenie, GOC:yaf Subtypes: positive regulation of striated muscle tissue development [GO:0045844], positive regulation of smooth muscle tissue development [GO:1905901] Also known as: up regulation of muscle tissue development, up-regulation of muscle tissue development, upregulation of muscle tissue development, activation of muscle tissue development Relationships: is a type of GO:0051094; is a type of regulation of muscle tissue development [GO:1901861]; positively regulates muscle tissue development [GO:0060537] Definition: Any process that activates or increases the frequency, rate or extent of muscle tissue development.